{
  "term_id": "GO:0031083",
  "gene_symbol": "BCAS4",
  "gene": "UniProtKB:Q8TDM0",
  "gene_name": "Breast carcinoma-amplified sequence 4",
  "term_label": "BLOC-1 complex"
}